{
  "gene": "UniProtKB:Q7Z3B1",
  "gene_name": "Neuronal growth regulator 1",
  "term_label": "heterophilic cell-cell adhesion",
  "term_id": "GO:0007157",
  "gene_symbol": "NEGR1"
}